{
  "term_id": "UNKNOWN:0003",
  "term_label": "Unknown cellular component",
  "gene_symbol": "MDGA2",
  "gene_name": "MAM domain-containing glycosylphosphatidylinositol anchor protein 2",
  "gene": "UniProtKB:Q7Z553"
}